saturated monocarboxylic acid metabolic process [GO:0032788] (biological process) Definition: The chemical reactions and pathways involving saturated monocarboxylic acids, any organic acid containing one carboxyl (COOH) group or anion (COO-) and fully saturated C-C bonds. Sources: GOC:mah, GOC:vk Also known as: saturated monocarboxylate metabolic process, saturated monocarboxylic acid metabolism Relationships: is a type of carboxylic acid metabolic process [GO:0019752]